{
  "gene": "UniProtKB:P32246",
  "gene_symbol": "CCR1",
  "term_id": "GO:0007204",
  "gene_name": "C-C chemokine receptor type 1",
  "term_label": "positive regulation of cytosolic calcium ion concentration"
}